{
  "term_label": "lipid transport",
  "gene_name": "Cholesterol transporter ABCA5",
  "gene": "UniProtKB:Q8WWZ7",
  "gene_symbol": "ABCA5",
  "term_id": "GO:0006869"
}